{
  "term_id": "GO:0005634",
  "term_label": "nucleus",
  "gene": "UniProtKB:Q96T25",
  "gene_name": "Zinc finger protein ZIC 5",
  "gene_symbol": "ZIC5"
}